{
  "term_id": "UNKNOWN:0002",
  "gene": "UniProtKB:Q9NZU0",
  "gene_symbol": "FLRT3",
  "gene_name": "Leucine-rich repeat transmembrane protein FLRT3",
  "term_label": "Unknown biological process"
}